{
  "gene_symbol": "IL36G",
  "gene": "UniProtKB:Q9NZH8",
  "term_id": "GO:0019221",
  "term_label": "cytokine-mediated signaling pathway",
  "gene_name": "Interleukin-36 gamma"
}